thiamine pyrophosphate transmembrane transporter activity [GO:0090422] (molecular function) Definition: Enables the transfer of thiamine pyrophosphate a substance from one side of a membrane to the other. Sources: GOC:tb Also known as: thiamine diphosphate transporter activity, thiamine pyrophosphate transporter activity Relationships: is a type of GO:0015234; is a type of organophosphate ester transmembrane transporter activity [GO:0015605]; is_a quaternary ammonium group transmembrane transporter activity [GO:0015651]; is part of thiamine pyrophosphate transmembrane transport [GO:0030974]